{
  "gene_name": "Speedy protein E10",
  "gene_symbol": "SPDYE10",
  "term_label": "protein kinase binding",
  "gene": "UniProtKB:P0DUX0",
  "term_id": "GO:0019901"
}